{
  "gene_name": "Methyl-CpG-binding domain protein 3-like 2B",
  "gene": "UniProtKB:A0A1B0GVZ6",
  "term_id": "GO:0000122",
  "gene_symbol": "MBD3L2B",
  "term_label": "negative regulation of transcription by RNA polymerase II"
}